otolith formation [GO:0032475] (biological process) Relationships: is a type of GO:0048646; is part of otolith morphogenesis [GO:0032474] Definition: The process that gives rise to an otolith. This process pertains to the initial formation of a structure from unspecified parts. Sources: GOC:dgh